{
  "term_id": "GO:1903489",
  "gene_name": "Prolactin",
  "term_label": "positive regulation of lactation",
  "gene_symbol": "PRL",
  "gene": "UniProtKB:P01236"
}